{
  "term_label": "centrosome",
  "term_id": "GO:0005813",
  "gene_name": "Centrosomal protein kizuna",
  "gene": "UniProtKB:Q2M2Z5",
  "gene_symbol": "KIZ"
}